iron-sulfur-molybdenum cofactor metabolic process [GO:1901286] (biological process) Subtypes: iron-sulfur-molybdenum cofactor catabolic process [GO:1901287], iron-sulfur-molybdenum cofactor biosynthetic process [GO:1901288] Also known as: FeMo-co metabolic process, FeMo-co metabolism, iron-molybdenum cofactor metabolic process, iron-molybdenum cofactor metabolism, iron-sulfur-molybdenum cofactor metabolism Relationships: is a type of metabolic process [GO:0008152] Definition: The chemical reactions and pathways involving iron-sulfur-molybdenum cofactor. Sources: GOC:TermGenie, GOC:yaf, UniPathway:UPA00782